acyl-phosphate-hexose phosphotransferase activity [GO:0047328] (molecular function) Relationships: is_a kinase activity [GO:0016301]; is a type of phosphotransferase activity, alcohol group as acceptor [GO:0016773] Also known as: acyl-phosphate:D-hexose phosphotransferase activity, hexose phosphate:hexose phosphotransferase activity Sources: EC:2.7.1.61, MetaCyc:2.7.1.61-RXN Definition: Catalysis of the reaction: D-hexose + acyl phosphate = D-hexose phosphate + an acid.